{
  "gene_name": "E3 ubiquitin-protein ligase ARIH2",
  "gene": "UniProtKB:O95376",
  "term_label": "ubiquitin conjugating enzyme binding",
  "gene_symbol": "ARIH2",
  "term_id": "GO:0031624"
}